{
  "gene_symbol": "ITGB1",
  "term_id": "GO:0007160",
  "term_label": "cell-matrix adhesion",
  "gene": "UniProtKB:P05556",
  "gene_name": "Integrin beta-1"
}